{
  "term_label": "cytoplasm",
  "gene_name": "Phospholipase A and acyltransferase 4",
  "gene_symbol": "PLAAT4",
  "gene": "UniProtKB:Q9UL19",
  "term_id": "GO:0005737"
}